{
  "gene": "UniProtKB:Q8N568",
  "gene_symbol": "DCLK2",
  "term_id": "GO:0005737",
  "gene_name": "Serine_threonine-protein kinase DCLK2",
  "term_label": "cytoplasm"
}